head kidney morphogenesis [GO:0072115] (biological process) Definition: The process in which the anatomical structures of the head kidney are generated and organized. The head kidney is a pronephros that consists of fused bilateral lobes located in the anterior part of the kidney. Sources: GOC:mtg_kidney_jan10, ZFA:0000669 Relationships: is a type of pronephros morphogenesis [GO:0072114]; is part of head kidney development [GO:0072113]